{
  "gene_symbol": "RPS9",
  "term_id": "GO:0042274",
  "term_label": "ribosomal small subunit biogenesis",
  "gene_name": "Small ribosomal subunit protein uS4",
  "gene": "UniProtKB:P46781"
}